{
  "term_label": "fatty acid beta-oxidation using acyl-CoA oxidase",
  "gene": "UniProtKB:Q15067",
  "gene_name": "Peroxisomal acyl-coenzyme A oxidase 1",
  "term_id": "GO:0033540",
  "gene_symbol": "ACOX1"
}